{
  "gene_name": "Tumor necrosis factor receptor superfamily member 27",
  "gene_symbol": "EDA2R",
  "term_label": "plasma membrane",
  "term_id": "GO:0005886",
  "gene": "UniProtKB:Q9HAV5"
}